{
  "gene_symbol": "EPB41L3",
  "term_label": "Unknown molecular function",
  "gene": "UniProtKB:Q9Y2J2",
  "term_id": "UNKNOWN:0001",
  "gene_name": "Band 4.1-like protein 3"
}